RNA polymerase II CTD heptapeptide repeat S7 phosphatase activity [GO:0180008] (molecular function) Definition: Catalysis of the reaction: RNA polymerase II large subunit CTD heptapeptide repeat--phospho-L-serine (consensus YSPTSPS)(position 7) + H2O = RNA polymerase II large subunit + phosphate. References: PMID:22622228 Relationships: is a type of RNA polymerase II CTD heptapeptide repeat phosphatase activity [GO:0008420] Also known as: RNA polymerase II C-terminal domain S7 phosphatase activity